cis-dihydroethylcatechol dehydrogenase activity [GO:0018519] (MF) Definition: Catalysis of the reaction: cis-1,2-dihydro-3-ethylcatechol + NAD+ = 3-ethylcatechol + H+ + NADH. Sources: EC:1.3.1.66, RHEA:18101 Also known as: cis-ethylbenzene glycol dehydrogenase activity, cis-1,2-dihydro-3-ethylcatechol:NAD+ oxidoreductase activity Relationships: is a type of GO:0016628